purine nucleoside monophosphate metabolic process [GO:0009126] (biological process) Definition: The chemical reactions and pathways involving purine nucleoside monophosphate, a compound consisting of a purine base linked to a ribose or deoxyribose sugar esterified with phosphate on the sugar. Also known as: purine nucleoside monophosphate metabolism Relationships: is a type of nucleoside monophosphate metabolic process [GO:0009123] Sources: GOC:go_curators, ISBN:0198506732 Subtypes: GO:0009127, purine nucleoside monophosphate catabolic process [GO:0009128], purine ribonucleoside monophosphate metabolic process [GO:0009167], GO:0009170